{
  "gene_symbol": "ZNF831",
  "term_id": "UNKNOWN:0003",
  "gene_name": "Zinc finger protein 831",
  "gene": "UniProtKB:Q5JPB2",
  "term_label": "Unknown cellular component"
}